{
  "gene_name": "PRKR-interacting protein 1",
  "term_id": "UNKNOWN:0002",
  "term_label": "Unknown biological process",
  "gene": "UniProtKB:Q9H875",
  "gene_symbol": "PRKRIP1"
}